{
  "gene_symbol": "MT3",
  "gene_name": "Metallothionein-3",
  "term_label": "cellular response to copper ion",
  "gene": "UniProtKB:P25713",
  "term_id": "GO:0071280"
}